{
  "gene_name": "La-related protein 6",
  "gene": "UniProtKB:Q9BRS8",
  "term_id": "GO:0005634",
  "gene_symbol": "LARP6",
  "term_label": "nucleus"
}